{
  "term_label": "odorant binding",
  "gene_symbol": "OR9K2",
  "term_id": "GO:0005549",
  "gene_name": "Olfactory receptor 9K2",
  "gene": "UniProtKB:Q8NGE7"
}